{
  "term_label": "metalloendopeptidase inhibitor activity",
  "gene": "UniProtKB:P16035",
  "gene_symbol": "TIMP2",
  "term_id": "GO:0008191",
  "gene_name": "Metalloproteinase inhibitor 2"
}